{
  "gene": "UniProtKB:Q9NRQ2",
  "term_id": "GO:0017128",
  "gene_name": "Phospholipid scramblase 4",
  "term_label": "phospholipid scramblase activity",
  "gene_symbol": "PLSCR4"
}